{
  "gene_name": "Histone H3.1t",
  "term_id": "GO:0000786",
  "gene_symbol": "H3-4",
  "term_label": "nucleosome",
  "gene": "UniProtKB:Q16695"
}